{
  "term_id": "GO:0008083",
  "gene_name": "Fibroblast growth factor 17",
  "term_label": "growth factor activity",
  "gene_symbol": "FGF17",
  "gene": "UniProtKB:O60258"
}